{
  "gene_name": "Inner centromere protein",
  "term_id": "GO:0051257",
  "gene_symbol": "INCENP",
  "gene": "UniProtKB:Q9NQS7",
  "term_label": "meiotic spindle midzone assembly"
}